positive regulation of bleb assembly [GO:1904172] (biological process) Relationships: is_a GO:0120034; is a type of regulation of bleb assembly [GO:1904170]; positively regulates bleb assembly [GO:0032060] References: PMID:25651887 Sources: GOC:TermGenie, GOC:als, GO_REF:0000058 Also known as: positive regulation of cell blebbing, up regulation of bleb assembly, up regulation of cell blebbing, up-regulation of bleb assembly, up-regulation of cell blebbing, upregulation of bleb assembly, upregulation of cell blebbing, activation of bleb assembly, activation of cell blebbing Definition: Any process that activates or increases the frequency, rate or extent of bleb assembly.